bacillithiol biosynthetic process [GO:0071793] (biological process) Definition: The chemical reactions and pathways resulting in the formation of bacillithiol, the alpha-anomeric glycoside of L-cysteinyl-D-glucosamine with L-malic acid. Bacillithiol, produced widely in the Firmicutes and sporadically in other bacterial lineages, is a low-molecular-weight thiol analogous to mycothiol in the Actinomycetes and glutathione in many species. Also known as: bacillithiol anabolism, bacillithiol biosynthesis, bacillithiol formation, bacillithiol synthesis References: PMID:20308541 Sources: GOC:dh Relationships: is a type of glycoside biosynthetic process [GO:0016138]; is a type of sulfur compound biosynthetic process [GO:0044272]; is a type of carboxylic acid biosynthetic process [GO:0046394]